{
  "gene_symbol": "ATG5",
  "gene": "UniProtKB:Q9H1Y0",
  "term_id": "GO:0000423",
  "term_label": "mitophagy",
  "gene_name": "Autophagy protein 5"
}